{
  "term_label": "cytoplasm",
  "gene": "UniProtKB:O94913",
  "gene_symbol": "PCF11",
  "gene_name": "Pre-mRNA cleavage complex 2 protein Pcf11",
  "term_id": "GO:0005737"
}